regulation of response to reactive oxygen species [GO:1901031] (biological process) Subtypes: negative regulation of response to reactive oxygen species [GO:1901032], positive regulation of response to reactive oxygen species [GO:1901033], regulation of removal of superoxide radicals [GO:2000121] Definition: Any process that modulates the frequency, rate or extent of response to reactive oxygen species. Sources: GOC:TermGenie, GOC:kmv Also known as: regulation of response to AOS, regulation of response to ROI, regulation of response to ROS, regulation of response to active oxygen species, regulation of response to reactive oxidative species, regulation of response to reactive oxygen intermediate Relationships: is a type of GO:1902882; regulates response to reactive oxygen species [GO:0000302]